neutral L-amino acid:sodium:chloride symporter activity [GO:0140931] (molecular function) Relationships: is a type of amino acid:sodium symporter activity [GO:0005283]; is a type of neutral L-amino acid transmembrane transporter activity [GO:0015175]; is a type of sodium:chloride symporter activity [GO:0015378] Also known as: neutral amino acid:sodium:chloride symporter activity Definition: Enables the transfer of a solute or solutes from one side of a membrane to the other according to the reaction: neutral L-amino acid(out) + Na+(out) + Cl-(out) = neutral L-amino acid(in) + Na+(in)+ Cl-(in). References: PMID:19478081